microtubule motor activity [GO:0003777] (molecular function) Definition: A motor activity that generates movement along a microtubule, driven by ATP hydrolysis. References: PMID:19686686, PMID:32684327, PMID:32842864 Relationships: is_a GO:0003774; is a type of polypeptide conformation or assembly isomerase activity [GO:0120544]; is a type of ATP-dependent activity [GO:0140657] Subtypes: minus-end-directed microtubule motor activity [GO:0008569], GO:0008574 Also known as: dynein, kinesin, ATP-dependent microtubule motor activity, axonemal motor activity, dynein ATPase activity, kinesin motor activity, kinetochore motor activity Note: Consider also annotating to the molecular function term 'microtubule binding ; GO:0008017'.